{
  "gene_symbol": "CLPSL2",
  "term_label": "Unknown biological process",
  "gene_name": "Colipase-like protein 2",
  "gene": "UniProtKB:Q6UWE3",
  "term_id": "UNKNOWN:0002"
}